{
  "gene_name": "Receptor-type tyrosine-protein phosphatase zeta",
  "gene_symbol": "PTPRZ1",
  "term_id": "UNKNOWN:0003",
  "term_label": "Unknown cellular component",
  "gene": "UniProtKB:P23471"
}